{
  "gene_symbol": "TLCD3A",
  "term_label": "lipid homeostasis",
  "term_id": "GO:0055088",
  "gene": "UniProtKB:Q8TBR7",
  "gene_name": "TLC domain-containing protein 3A"
}